{
  "term_label": "Unknown molecular function",
  "term_id": "UNKNOWN:0001",
  "gene_name": "Actin maturation protease",
  "gene": "UniProtKB:Q5BKX5",
  "gene_symbol": "ACTMAP"
}